{
  "term_id": "GO:0031087",
  "term_label": "deadenylation-independent decapping of nuclear-transcribed mRNA",
  "gene_symbol": "EDC4",
  "gene_name": "Enhancer of mRNA-decapping protein 4",
  "gene": "UniProtKB:Q6P2E9"
}